carbonyl reductase (NADPH) activity [GO:0004090] (molecular function) Definition: Catalysis of the reaction: a secondary alcohol + NADP+ = a ketone + H+ + NADPH. Sources: RHEA:19257 Also known as: prostaglandin 9-ketoreductase activity, xenobiotic ketone reductase activity, ALR3, NADPH-dependent carbonyl reductase activity, NADPH2-dependent carbonyl reductase activity, aldehyde reductase 1, aldehyde reductase I activity, carbonyl reductase activity, nonspecific NADPH-dependent carbonyl reductase activity, secondary-alcohol:NADP+ oxidoreductase activity Relationships: is a type of GO:0008106